negative regulation of cell proliferation involved in heart morphogenesis [GO:2000137] (biological process) Definition: Any process that stops, prevents, or reduces the frequency, rate or extent of cell proliferation involved in heart morphogenesis. Sources: GOC:dph Subtypes: negative regulation of cell proliferation involved in heart valve morphogenesis [GO:0003252], negative regulation of cardioblast proliferation [GO:1905061] Relationships: is a type of negative regulation of cell population proliferation [GO:0008285]; is a type of regulation of cell proliferation involved in heart morphogenesis [GO:2000136]; negatively regulates cell proliferation involved in heart morphogenesis [GO:0061323]